pyruvate catabolic process [GO:0042867] (biological process) Also known as: pyruvate breakdown, pyruvate catabolism, pyruvate degradation Relationships: is a type of pyruvate metabolic process [GO:0006090]; is a type of GO:0072329 Definition: The chemical reactions and pathways resulting in the breakdown of pyruvate, 2-oxopropanoate. Subtypes: pyruvate fermentation [GO:0019660] Sources: GOC:go_curators